{
  "gene": "UniProtKB:Q8NEB9",
  "term_label": "phosphatidylinositol 3-kinase complex, class III, type II",
  "gene_name": "Phosphatidylinositol 3-kinase catalytic subunit type 3",
  "term_id": "GO:0034272",
  "gene_symbol": "PIK3C3"
}